small ribosomal subunit rRNA binding [GO:0070181] (molecular function) Sources: GOC:elh Definition: Binding to small ribosomal subunit RNA (SSU rRNA), a constituent of the small ribosomal subunit. In S. cerevisiae, this is the 18S rRNA. Relationships: is a type of rRNA binding [GO:0019843] Also known as: 18S rRNA binding, SSU rRNA binding